{
  "gene": "UniProtKB:Q14126",
  "term_id": "GO:0030057",
  "gene_name": "Desmoglein-2",
  "gene_symbol": "DSG2",
  "term_label": "desmosome"
}